{
  "gene_symbol": "PLPPR2",
  "gene_name": "Phospholipid phosphatase-related protein type 2",
  "term_label": "phospholipid dephosphorylation",
  "gene": "UniProtKB:Q96GM1",
  "term_id": "GO:0046839"
}